{
  "gene_symbol": "ZBTB25",
  "term_label": "regulation of cytokine production",
  "term_id": "GO:0001817",
  "gene": "UniProtKB:P24278",
  "gene_name": "Zinc finger and BTB domain-containing protein 25"
}